malonyl-CoA metabolic process [GO:2001293] (biological process) Definition: The chemical reactions and pathways involving malonyl-CoA, the S-malonyl derivative of coenzyme A. Also known as: malonyl-CoA metabolism Subtypes: malonyl-CoA catabolic process [GO:2001294], malonyl-CoA biosynthetic process [GO:2001295] References: PMID:11902724, PMID:15726818, PMID:18981598 Sources: GOC:yaf Relationships: is a type of GO:0006637